{
  "term_id": "GO:0003743",
  "gene_name": "Translation initiation factor eIF-2B subunit alpha",
  "gene": "UniProtKB:Q14232",
  "gene_symbol": "EIF2B1",
  "term_label": "translation initiation factor activity"
}